{
  "term_id": "UNKNOWN:0002",
  "gene_name": "Alanine aminotransferase 2",
  "term_label": "Unknown biological process",
  "gene": "UniProtKB:Q8TD30",
  "gene_symbol": "GPT2"
}